{
  "gene_symbol": "PPP1R3C",
  "term_id": "GO:0008157",
  "gene": "UniProtKB:Q9UQK1",
  "gene_name": "Protein phosphatase 1 regulatory subunit 3C",
  "term_label": "protein phosphatase 1 binding"
}